penicillin amidase activity [GO:0008953] (molecular function) Also known as: palmitoleoyl [acyl-carrier protein]-dependent acyltransferase activity, alpha-acylamino-beta-lactam acylhydrolase activity, ampicillin acylase activity, benzylpenicillin acylase activity, novozym 217, penicillin acylase activity, penicillin amidohydrolase activity, semacylase activity Relationships: is a type of hydrolase activity, acting on carbon-nitrogen (but not peptide) bonds, in linear amides [GO:0016811] Definition: Catalysis of the reaction: penicillin + H2O = a carboxylate + 6-aminopenicillanate. Sources: EC:3.5.1.11